{
  "term_label": "non-motile cilium",
  "gene_symbol": "NPHP4",
  "term_id": "GO:0097730",
  "gene": "UniProtKB:O75161",
  "gene_name": "Nephrocystin-4"
}